thiamine transmembrane transporter activity [GO:0015234] (molecular function) Sources: GOC:ai, GOC:mtg_transport, ISBN:0815340729 Definition: Enables the transfer of thiamine from one side of a membrane to the other. Thiamine is vitamin B1, a water soluble vitamin present in fresh vegetables and meats, especially liver. Relationships: is a type of GO:0090482; is a type of azole transmembrane transporter activity [GO:1901474]; is_a sulfur compound transmembrane transporter activity [GO:1901682]; BFO_0000050 thiamine transmembrane transport [GO:0071934] Subtypes: thiamine:proton symporter activity [GO:0034215], ABC-type thiamine transporter activity [GO:0048502], thiamine pyrophosphate transmembrane transporter activity [GO:0090422] Also known as: thiamin permease activity, thiamin transmembrane transporter activity, thiamine permease activity, vitamin B1 transporter activity, thiamin uptake transporter activity, thiamine uptake transmembrane transporter activity